light-activated voltage-gated calcium channel activity [GO:0008086] (molecular function) Sources: GOC:mtg_transport Definition: Enables the transmembrane transfer of a calcium ion by a voltage-gated channel that is activated in response to light. A voltage-gated channel is a channel whose open state is dependent on the voltage across the membrane in which it is embedded. Relationships: is a type of voltage-gated calcium channel activity [GO:0005245]; is a type of light-activated monoatomic ion channel activity [GO:0010461]; is part of calcium-mediated signaling [GO:0019722] Also known as: light-activated voltage gated calcium channel activity, light-activated voltage-dependent calcium channel activity